protein tetramerization [GO:0051262] (biological process) Regulation: regulated by regulation of protein tetramerization [GO:1901090]; negatively regulated by negative regulation of protein tetramerization [GO:1901091]; positively regulated by positive regulation of protein tetramerization [GO:1901092] Relationships: is a type of GO:0051259 Also known as: protein tetramer assembly, protein tetramer biosynthesis, protein tetramer biosynthetic process, protein tetramer formation Subtypes: protein homotetramerization [GO:0051289], protein heterotetramerization [GO:0051290] Definition: The formation of a protein tetramer, a macromolecular structure consisting of four noncovalently associated identical or nonidentical subunits. Sources: GOC:ecd